SL snRNP [GO:0071024] (cellular component) Sources: GOC:krc, ISBN:0879697393 Relationships: is a type of GO:0097525 Definition: A ribonucleoprotein complex that contains spliced leader (SL) RNA and associated proteins.